{
  "gene": "UniProtKB:Q9HDC5",
  "gene_symbol": "JPH1",
  "gene_name": "Junctophilin-1",
  "term_id": "UNKNOWN:0001",
  "term_label": "Unknown molecular function"
}